{
  "term_id": "GO:0000226",
  "term_label": "microtubule cytoskeleton organization",
  "gene_name": "Alpha-tubulin N-acetyltransferase 1",
  "gene_symbol": "ATAT1",
  "gene": "UniProtKB:Q5SQI0"
}